{
  "gene": "UniProtKB:O60245",
  "gene_name": "Protocadherin-7",
  "gene_symbol": "PCDH7",
  "term_id": "GO:0005886",
  "term_label": "plasma membrane"
}